{
  "gene_name": "Very-long-chain enoyl-CoA reductase",
  "gene_symbol": "TECR",
  "gene": "UniProtKB:Q9NZ01",
  "term_label": "very-long-chain enoyl-CoA reductase activity",
  "term_id": "GO:0102758"
}